{
  "term_id": "UNKNOWN:0001",
  "gene": "UniProtKB:A0A494C0Y3",
  "gene_name": "Protein FAM246A",
  "term_label": "Unknown molecular function",
  "gene_symbol": "FAM246A"
}